{
  "term_id": "GO:0005634",
  "gene_symbol": "HMBOX1",
  "gene_name": "Homeobox-containing protein 1",
  "gene": "UniProtKB:Q6NT76",
  "term_label": "nucleus"
}